{
  "gene_name": "CCHC-type zinc finger nucleic acid binding protein",
  "gene": "UniProtKB:P62633",
  "gene_symbol": "CNBP",
  "term_label": "translation regulator activity",
  "term_id": "GO:0045182"
}